perithecium formation [GO:0106154] (biological process) Definition: The process of producing flask-shaped fruiting bodies, called perithecia. In the ascomycetous fungi such as Neurospora crassa and Sordaria macrospora, these perithecia are formed in the sexual phase and they discharge ascospores through the ostiolum at the tip of the perithecial neck. Relationships: is a type of perithecium development [GO:0120165] References: PMID:19547974, PMID:21134480, PMID:25311923 Sources: DOI:10.1007/978-3-642-00286-1_2, GOC:ach